{
  "term_label": "synaptic transmission, GABAergic",
  "gene_name": "Gamma-aminobutyric acid receptor subunit gamma-3",
  "term_id": "GO:0051932",
  "gene_symbol": "GABRG3",
  "gene": "UniProtKB:Q99928"
}